{
  "gene_symbol": "HBE1",
  "term_id": "GO:0031838",
  "gene_name": "Hemoglobin subunit epsilon",
  "term_label": "haptoglobin-hemoglobin complex",
  "gene": "UniProtKB:P02100"
}